regulation of dipeptide transport [GO:0090089] (biological process) Sources: GOC:dph, GOC:tb Relationships: is a type of GO:0090088; regulates dipeptide transport [GO:0042938] Definition: Any process that modulates the rate, frequency or extent of dipeptide transport. Dipeptide transport is the directed movement of a dipeptide, a combination of two amino acids by means of a peptide (-CO-NH-) link, into, out of or within a cell, or between cells, by means of some agent such as a transporter or pore. Subtypes: negative regulation of dipeptide transport [GO:2000879], positive regulation of dipeptide transport [GO:2000880], regulation of dipeptide transmembrane transport [GO:2001148]